{
  "term_label": "mitotic recombination",
  "gene_name": "DNA repair protein RAD52 homolog",
  "term_id": "GO:0006312",
  "gene": "UniProtKB:P43351",
  "gene_symbol": "RAD52"
}